{
  "term_label": "Unknown molecular function",
  "term_id": "UNKNOWN:0001",
  "gene_symbol": "C8B",
  "gene": "UniProtKB:P07358",
  "gene_name": "Complement component C8 beta chain"
}